SIN/MEN signaling complex [GO:0160065] (CC) Relationships: is a type of protein-containing complex [GO:0032991]; is part of outer plaque of mitotic spindle pole body [GO:0061499] Definition: A protein complex associated with the mitotic spindle pole body during interphase and mitosis and comprises of the proteins of the septation initiation signaling network (SIN) of fission yeast or mitotic exit network (MEN) of budding yeast, organized by two scaffold/adaptor proteins. Also known as: SIN/MEN signalling complex, Hippo signaling complex, MEN signaling complex, SIN signaling complex References: PMID:21131906, PMID:22525225, PMID:22684255 Subtypes: interphase SIN signaling complex [GO:0160066], new spindle pole body SIN signaling complex [GO:0160067]